L-histidine biosynthetic process [GO:0000105] (biological process) Definition: The chemical reactions and pathways resulting in the formation of L-histidine, 2-amino-3-(1H-imidazol-4-yl)propanoic acid. Sources: GOC:go_curators Regulation: regulated by regulation of histidine biosynthetic process [GO:0120213]; negatively regulated by negative regulation of histidine biosynthetic process [GO:0120214]; positively regulated by positive regulation of histidine biosynthetic process [GO:0120215] Also known as: histidine biosynthetic process, histidine anabolism, histidine biosynthesis, histidine formation, histidine synthesis Relationships: is a type of L-histidine metabolic process [GO:0006547]; is a type of aromatic amino acid family biosynthetic process [GO:0009073]; is a type of L-amino acid biosynthetic process [GO:0170034]; is a type of proteinogenic amino acid biosynthetic process [GO:0170038]